positive regulation of protein localization to kinetochore [GO:1905342] (biological process) Also known as: positive regulation of protein localisation to kinetochore, up regulation of protein localisation to kinetochore, up regulation of protein localization to kinetochore, up-regulation of protein localisation to kinetochore, up-regulation of protein localization to kinetochore, upregulation of protein localisation to kinetochore, upregulation of protein localization to kinetochore, activation of condensin localization to kinetochore, activation of protein localisation to kinetochore, activation of protein localization to kinetochore, positive regulation of condensin localization to kinetochore, up regulation of condensin localization to kinetochore, up-regulation of condensin localization to kinetochore, upregulation of condensin localization to kinetochore Relationships: is a type of positive regulation of protein localization [GO:1903829]; is a type of regulation of protein localization to kinetochore [GO:1905340]; positively regulates GO:0034501 Subtypes: positive regulation of chromosome passenger complex localization to kinetochore [GO:0140430] Definition: Any process that activates or increases the frequency, rate or extent of protein localization to kinetochore. References: PMID:22581055 Sources: GOC:TermGenie, GO_REF:0000058 Note: Q9H211 in Human in PMID:22581055